mitotic cytokinesis checkpoint signaling [GO:0044878] (biological process) Relationships: is a type of GO:0007093; is a type of GO:0010972 Also known as: mitotic cytokinesis checkpoint, signal transduction involved in mitotic cytokinesis checkpoint, signaling pathway involved in mitotic cytokinesis checkpoint, signalling cascade involved in mitotic cytokinesis checkpoint, cytokinesis after mitosis checkpoint, defective cytokinesis checkpoint, signalling pathway involved in mitotic cytokinesis checkpoint References: PMID:17538026 Sources: GOC:jl, GOC:mtg_cell_cycle Definition: A signaling process that contributes to a mitotic cell cycle checkpoint that detects a defect in cytokinesis and prevents further rounds of nuclear division until cytokinesis is completed.